{
  "term_label": "visual perception",
  "term_id": "GO:0007601",
  "gene_name": "Protocadherin-15",
  "gene_symbol": "PCDH15",
  "gene": "UniProtKB:Q96QU1"
}